maternal determination of dorsal/ventral axis, ovarian follicular epithelium, germ-line encoded [GO:0008070] (BP) Definition: Polarization of the ovarian follicle cells along the dorsal-ventral axis by a gene product encoded by cells of the germ line. Sources: GOC:mtg_sensu, ISBN:0879694238 Also known as: maternal determination of dorsal-ventral axis, ovarian follicular epithelium, germ-line encoded, maternal determination of dorsoventral axis, ovarian follicular epithelium, germ-line encoded Relationships: is a type of dorsal/ventral axis specification, ovarian follicular epithelium [GO:0008069]